{
  "gene_symbol": "KCNMB2",
  "term_id": "GO:0008076",
  "gene_name": "Calcium-activated potassium channel subunit beta-2",
  "term_label": "voltage-gated potassium channel complex",
  "gene": "UniProtKB:Q9Y691"
}